P-type sodium:potassium-exchanging transporter activity [GO:0005391] (molecular function) Subtypes: P-type sodium:potassium-exchanging transporter activity involved in regulation of cardiac muscle cell membrane potential [GO:0086037] Relationships: is a type of P-type sodium transporter activity [GO:0008554]; is a type of GO:0008556; is part of establishment or maintenance of transmembrane electrochemical gradient [GO:0010248] Sources: EC:7.2.2.13 Also known as: sodium pump, P-type sodium:potassium-exchanging ATPase activity, sodium/potassium-exchanging ATPase activity, sodium/potassium-transporting ATPase activity, sodium:potassium exchanging ATPase activity, sodium:potassium-exchanging ATPase activity, Na(+)/K(+)-ATPase activity, Na(+)/K(+)-exchanging ATPase activity, Na+,K+-ATPase activity, Na+/K+-ATPase activity, Na+/K+-exchanging ATPase activity, Na,K-activated ATPase activity Definition: Enables the transfer of a solute or solutes from one side of a membrane to the other according to the reaction: ATP + H2O + Na+(in) + K+(out) = ADP + phosphate + Na+(out) + K+(in). Regulation: regulated by regulation of P-type sodium:potassium-exchanging transporter activity [GO:1903406]; negatively regulated by GO:1903407; positively regulated by positive regulation of P-type sodium:potassium-exchanging transporter activity [GO:1903408]